cyclic-di-AMP phosphodiesterase activity [GO:0106409] (molecular function) Relationships: is a type of nucleotidyltransferase activity [GO:0016779] Definition: Catalysis of the reaction: 3',3'-c-di-AMP + H2O = 5'-O-phosphonoadenylyl-(3'-5')-adenosine + H+. References: PMID:21909268 Sources: RHEA:54420